positive regulation of peptidyl-serine phosphorylation of STAT protein [GO:0033141] (biological process) Relationships: is a type of positive regulation of peptidyl-serine phosphorylation [GO:0033138]; is a type of regulation of peptidyl-serine phosphorylation of STAT protein [GO:0033139]; positively regulates serine phosphorylation of STAT protein [GO:0042501] Definition: Any process that activates or increases the frequency, rate or extent of the phosphorylation of a serine residue of a STAT (Signal Transducer and Activator of Transcription) protein. Also known as: activation of serine phosphorylation of STAT3 protein, positive regulation of serine phosphorylation of STAT3 protein, up regulation of serine phosphorylation of STAT3 protein, up-regulation of serine phosphorylation of STAT3 protein, upregulation of serine phosphorylation of STAT3 protein Sources: GOC:mah